{
  "term_label": "neuronal cell body",
  "gene": "UniProtKB:Q9GZP1",
  "gene_name": "Neurensin-2",
  "gene_symbol": "NRSN2",
  "term_id": "GO:0043025"
}